{
  "gene_name": "DnaJ homolog subfamily C member 28",
  "term_label": "Unknown molecular function",
  "gene_symbol": "DNAJC28",
  "gene": "UniProtKB:Q9NX36",
  "term_id": "UNKNOWN:0001"
}